{
  "gene_name": "Ectodysplasin-A receptor-associated adapter protein",
  "term_id": "UNKNOWN:0002",
  "term_label": "Unknown biological process",
  "gene": "UniProtKB:Q8WWZ3",
  "gene_symbol": "EDARADD"
}